{
  "gene_symbol": "KCNIP3",
  "gene_name": "Calsenilin",
  "term_id": "GO:0015459",
  "term_label": "potassium channel regulator activity",
  "gene": "UniProtKB:Q9Y2W7"
}